gamma-glutamylaminecyclotransferase activity [GO:0061929] (molecular function) Relationships: is a type of amidine-lyase activity [GO:0016842] Definition: Catalysis of the reaction: epsilon-(L-gamma-glutamyl)-L-lysine = L-lysine + 5-oxo-L-proline. References: PMID:20110353, PMID:6107907